tyrosyl-tRNA aminoacylation [GO:0006437] (biological process) Sources: GOC:mcc, ISBN:0716730510 Definition: The process of coupling tyrosine to tyrosyl-tRNA, catalyzed by tyrosyl-tRNA synthetase. The tyrosyl-tRNA synthetase is a class-I synthetase. The activated amino acid is transferred to the 2'-OH group of a tyrosine-accetping tRNA. The 2'-O-aminoacyl-tRNA will ultimately migrate to the 3' position via transesterification. Relationships: is_a tRNA aminoacylation for protein translation [GO:0006418] Subtypes: GO:0070184